{
  "term_label": "serine palmitoyltransferase complex",
  "term_id": "GO:0017059",
  "gene": "UniProtKB:Q9P0S3",
  "gene_symbol": "ORMDL1",
  "gene_name": "ORM1-like protein 1"
}